{
  "gene_name": "MANSC domain-containing protein 4",
  "gene": "UniProtKB:A6NHS7",
  "term_id": "GO:0060429",
  "gene_symbol": "MANSC4",
  "term_label": "epithelium development"
}